{
  "gene_name": "ETS domain-containing protein Elk-1",
  "gene_symbol": "ELK1",
  "term_id": "GO:0005634",
  "term_label": "nucleus",
  "gene": "UniProtKB:P19419"
}